{
  "gene_symbol": "ABCC8",
  "term_id": "GO:0140359",
  "term_label": "ABC-type transporter activity",
  "gene": "UniProtKB:Q09428",
  "gene_name": "ATP-binding cassette sub-family C member 8"
}